glycerol-3-phosphate dehydrogenase [NAD(P)+] activity [GO:0047952] (molecular function) Relationships: is a type of GO:0016616 References: PMID:28326 Sources: EC:1.1.1.94 Also known as: L-alpha-glycerol phosphate dehydrogenase activity, L-alpha-glycerophosphate dehydrogenase activity, L-glycerol phosphate dehydrogenase activity, L-glycerophosphate dehydrogenase activity, hydroglycerophosphate dehydrogenase activity, glycerol phosphate dehydrogenase (nicotinamide adenine dinucleotide (phosphate)) activity, glycerol-3-phosphate dehydrogenase (NAD(P)+) activity, L-glycerol-3-phosphate:NAD(P) oxidoreductase activity, sn-glycerol-3-phosphate:NAD(P)+ 2-oxidoreductase activity Subtypes: glycerol-3-phosphate dehydrogenase (NAD+) activity [GO:0141152], GO:0141153 Definition: Catalysis of the reaction: sn-glycerol 3-phosphate + NAD(P)+ = glycerone phosphate + NAD(P)H + H+.